{
  "term_label": "proteasome-mediated ubiquitin-dependent protein catabolic process",
  "gene_symbol": "RAD23A",
  "gene_name": "UV excision repair protein RAD23 homolog A",
  "term_id": "GO:0043161",
  "gene": "UniProtKB:P54725"
}